{
  "gene": "UniProtKB:P0CB47",
  "term_id": "GO:0006360",
  "term_label": "transcription by RNA polymerase I",
  "gene_name": "Upstream-binding factor 1-like protein 1",
  "gene_symbol": "UBTFL1"
}